{
  "gene_name": "Tumor necrosis factor ligand superfamily member 4",
  "gene": "UniProtKB:P23510",
  "term_id": "GO:0032813",
  "gene_symbol": "TNFSF4",
  "term_label": "tumor necrosis factor receptor superfamily binding"
}